{
  "gene_name": "Endoribonuclease ZC3H12A",
  "gene": "UniProtKB:Q5D1E8",
  "term_id": "GO:0005634",
  "gene_symbol": "ZC3H12A",
  "term_label": "nucleus"
}